positive regulation of conidium formation [GO:0075307] (biological process) Sources: GOC:di, GOC:pamgo_curators Relationships: is a type of positive regulation of cell development [GO:0010720]; is a type of GO:0043938; is a type of regulation of conidium formation [GO:0075306]; is a type of positive regulation of asexual reproduction [GO:1903666]; RO_0002213 conidium formation [GO:0048315] Definition: Any process that activates, maintains or increases the frequency, rate or extent of conidium formation, a process of producing non-motile spores, called conidia, via mitotic asexual reproduction in higher fungi. Conidia are haploid cells genetically identical to their haploid parent. They are produced by conversion of hyphal elements, or are borne on sporogenous cells on or within specialized structures termed conidiophores, and participate in dispersal of the fungus.